{
  "gene_symbol": "ADGRL4",
  "gene_name": "Adhesion G protein-coupled receptor L4",
  "term_id": "GO:0005886",
  "gene": "UniProtKB:Q9HBW9",
  "term_label": "plasma membrane"
}